{
  "term_label": "translation elongation factor activity",
  "term_id": "GO:0003746",
  "gene_symbol": "EIF5A2",
  "gene_name": "Eukaryotic translation initiation factor 5A-2",
  "gene": "UniProtKB:Q9GZV4"
}